{
  "term_label": "Unknown molecular function",
  "gene_name": "Multiple myeloma tumor-associated protein 2",
  "gene_symbol": "MMTAG2",
  "gene": "UniProtKB:Q9BU76",
  "term_id": "UNKNOWN:0001"
}